{
  "term_id": "GO:0003729",
  "term_label": "mRNA binding",
  "gene": "UniProtKB:Q7Z739",
  "gene_name": "YTH domain-containing family protein 3",
  "gene_symbol": "YTHDF3"
}